positive regulation of aggregation involved in sorocarp development [GO:0110013] (biological process) References: PMID:28257811 Sources: GOC:rjd Relationships: is a type of positive regulation of response to nutrient levels [GO:0032109]; is a type of positive regulation of cellular process [GO:0048522]; is_a GO:0051094; is a type of regulation of aggregation involved in sorocarp development [GO:0060176]; positively regulates aggregation involved in sorocarp development [GO:0031152] Definition: Any process that increases the frequency, rate or extent of aggregation involved in sorocarp development. Aggregation involved in sorocarp development is the process whose specific outcome is the progression of the aggregate over time, from its formation to the point when a slug is formed. Aggregate development begins in response to starvation and continues by the chemoattractant-mediated movement of cells toward each other. The aggregate is a multicellular structure that gives rise to the slug.